{
  "gene": "UniProtKB:Q6ZU15",
  "term_label": "molecular adaptor activity",
  "term_id": "GO:0060090",
  "gene_symbol": "SEPTIN14",
  "gene_name": "Septin-14"
}